{
  "gene_symbol": "MT1L",
  "gene_name": "Metallothionein-1L",
  "term_label": "metal ion binding",
  "gene": "UniProtKB:Q93083",
  "term_id": "GO:0046872"
}